{
  "term_label": "intracellular signal transduction",
  "gene": "UniProtKB:Q9Y243",
  "gene_symbol": "AKT3",
  "gene_name": "RAC-gamma serine_threonine-protein kinase",
  "term_id": "GO:0035556"
}